{
  "gene_name": "Melanoma-derived growth regulatory protein",
  "term_label": "Unknown molecular function",
  "gene": "UniProtKB:Q16674",
  "term_id": "UNKNOWN:0001",
  "gene_symbol": "MIA"
}